{
  "term_label": "axon",
  "gene_symbol": "SYT8",
  "gene": "UniProtKB:Q8NBV8",
  "gene_name": "Synaptotagmin-8",
  "term_id": "GO:0030424"
}